{
  "gene_symbol": "ESPNL",
  "term_id": "GO:0051015",
  "gene": "UniProtKB:Q6ZVH7",
  "term_label": "actin filament binding",
  "gene_name": "Espin-like protein"
}